{
  "gene_symbol": "FBLN5",
  "term_id": "GO:0048251",
  "gene": "UniProtKB:Q9UBX5",
  "term_label": "elastic fiber assembly",
  "gene_name": "Fibulin-5"
}